{
  "term_id": "GO:0070374",
  "gene_name": "Metallothionein-3",
  "gene": "UniProtKB:P25713",
  "term_label": "positive regulation of ERK1 and ERK2 cascade",
  "gene_symbol": "MT3"
}